sulfoquinovose isomerase activity [GO:0061593] (molecular function) Definition: Catalysis of the reaction: 6-sulfo-beta-D-quinovose = 6-deoxy-6-sulfo-D-fructose. References: PMID:24463506 Sources: RHEA:40439 Relationships: is_a intramolecular oxidoreductase activity, interconverting aldoses and ketoses [GO:0016861]